retinal cone cell apoptotic process [GO:0097474] (biological process) Also known as: cone photoreceptor apoptotic process Sources: CL:0000573, GOC:jc Definition: Any apoptotic process in a retinal cone cell, one of the two photoreceptor cell types of the vertebrate retina. Relationships: is a type of neuron apoptotic process [GO:0051402]; is a type of GO:1990009